acyl-lipid (n+3)-(Z)-desaturase (ferredoxin) activity [GO:0102850] (molecular function) Also known as: 1-18:1-2-16:0-phosphatidylglycerol omega-6 desaturase activity Sources: RHEA:46376 Definition: Catalysis of the reaction: a (9Z)-octadecenoyl-containing glycerolipid + 2 H+ + O2 + 2 reduced [2Fe-2S]-[ferredoxin] = a (9Z,12Z)-octadecadienoyl-containing glycerolipid + 2 H2O + 2 oxidized [2Fe-2S]-[ferredoxin]. Relationships: is a type of oxidoreductase activity, acting on paired donors, with oxidation of a pair of donors resulting in the reduction of molecular oxygen to two molecules of water [GO:0016717]